{
  "gene_symbol": "ZNF791",
  "term_label": "RNA polymerase II transcription regulatory region sequence-specific DNA binding",
  "term_id": "GO:0000977",
  "gene": "UniProtKB:Q3KP31",
  "gene_name": "Zinc finger protein 791"
}